{
  "term_label": "structural constituent of nuclear pore",
  "gene": "UniProtKB:P57740",
  "gene_name": "Nuclear pore complex protein Nup107",
  "term_id": "GO:0017056",
  "gene_symbol": "NUP107"
}